{
  "term_id": "GO:0001228",
  "term_label": "DNA-binding transcription activator activity, RNA polymerase II-specific",
  "gene_name": "Zinc finger protein 750",
  "gene": "UniProtKB:Q32MQ0",
  "gene_symbol": "ZNF750"
}